{
  "gene": "UniProtKB:Q8NGV0",
  "term_id": "GO:0005886",
  "term_label": "plasma membrane",
  "gene_name": "Olfactory receptor 2Y1",
  "gene_symbol": "OR2Y1"
}